regulation of blood coagulation [GO:0030193] (biological process) Definition: Any process that modulates the frequency, rate or extent of blood coagulation. Relationships: is a type of regulation of response to external stimulus [GO:0032101]; is a type of GO:0050818; is a type of regulation of wound healing [GO:0061041]; is a type of GO:1900046; regulates GO:0007596 Sources: GOC:mah Subtypes: positive regulation of blood coagulation [GO:0030194], negative regulation of blood coagulation [GO:0030195], GO:0051917, regulation of blood coagulation, common pathway [GO:2000260], regulation of blood coagulation, extrinsic pathway [GO:2000263], regulation of blood coagulation, intrinsic pathway [GO:2000266]